{
  "term_id": "GO:0000981",
  "gene_symbol": "DACH2",
  "term_label": "DNA-binding transcription factor activity, RNA polymerase II-specific",
  "gene_name": "Dachshund homolog 2",
  "gene": "UniProtKB:Q96NX9"
}